{
  "term_label": "developmental process",
  "gene": "UniProtKB:P21964",
  "gene_symbol": "COMT",
  "term_id": "GO:0032502",
  "gene_name": "Catechol O-methyltransferase"
}